{
  "gene_symbol": "MTOR",
  "term_label": "TORC1 signaling",
  "gene_name": "Serine_threonine-protein kinase mTOR",
  "term_id": "GO:0038202",
  "gene": "UniProtKB:P42345"
}